{
  "gene_name": "Putative inactive phosphatidylinositol 4-kinase alpha-like protein P1",
  "term_id": "UNKNOWN:0002",
  "term_label": "Unknown biological process",
  "gene_symbol": "PI4KAP1",
  "gene": "UniProtKB:Q8N8J0"
}